salt aversion [GO:0035199] (biological process) Sources: GOC:bf Relationships: is a type of GO:0007631; is part of response to chemical [GO:0042221] Definition: The specific avoidance actions or reactions of an organism in response to the perception of salt. Also known as: behavioral response to salt